cholest-5-ene-3-beta,7-alpha-diol 3-beta-dehydrogenase activity [GO:0047016] (molecular function) Also known as: 3beta-hydroxy-delta5-C27-steroid oxidoreductase, 3-beta-hydroxy-Delta(5)-C(27)-steroid oxidoreductase activity, cholest-5-ene-3beta,7alpha-diol 3beta-dehydrogenase activity, cholest-5-ene-3beta,7alpha-diol:NAD+ 3-oxidoreductase activity Definition: Catalysis of the reaction: NAD+ + 7-alpha-hydroxycholesterol = NADH + H+ + 7-alpha-hydroxycholest-4-en-3-one. Sources: EC:1.1.1.181, MetaCyc:1.1.1.181-RXN Relationships: is a type of GO:0016616